{
  "gene": "UniProtKB:P13164",
  "gene_name": "Interferon-induced transmembrane protein 1",
  "term_id": "UNKNOWN:0001",
  "gene_symbol": "IFITM1",
  "term_label": "Unknown molecular function"
}